{
  "gene_name": "Protein lifeguard 2",
  "term_id": "GO:1902042",
  "gene_symbol": "FAIM2",
  "term_label": "negative regulation of extrinsic apoptotic signaling pathway via death domain receptors",
  "gene": "UniProtKB:Q9BWQ8"
}